{
  "term_label": "proteolysis",
  "gene_symbol": "HTRA4",
  "term_id": "GO:0006508",
  "gene": "UniProtKB:P83105",
  "gene_name": "Serine protease HTRA4"
}